{
  "term_id": "UNKNOWN:0002",
  "gene_name": "Unconventional myosin-XVIIIa",
  "gene": "UniProtKB:Q92614",
  "gene_symbol": "MYO18A",
  "term_label": "Unknown biological process"
}